negative regulation of exosomal secretion [GO:1903542] (biological process) Definition: Any process that stops, prevents or reduces the frequency, rate or extent of exosomal secretion. Also known as: down regulation of exosomal secretion, down regulation of exosomal secretory pathway, down regulation of extracellular vesicular exosome secretion, down regulation of secretion of exosome, down-regulation of exosomal secretion, down-regulation of exosomal secretory pathway, down-regulation of extracellular vesicular exosome secretion, down-regulation of secretion of exosome, downregulation of exosomal secretion, downregulation of exosomal secretory pathway, downregulation of extracellular vesicular exosome secretion, downregulation of secretion of exosome, negative regulation of exosomal secretory pathway, negative regulation of extracellular vesicular exosome secretion, negative regulation of secretion of exosome, down regulation of exosomal protein secretion, down-regulation of exosomal protein secretion, downregulation of exosomal protein secretion, inhibition of exosomal protein secretion, inhibition of exosomal secretion, inhibition of exosomal secretory pathway, inhibition of extracellular vesicular exosome secretion, inhibition of secretion of exosome, negative regulation of exosomal protein secretion Relationships: is a type of negative regulation of exocytosis [GO:0045920]; is a type of regulation of exosomal secretion [GO:1903541]; negatively regulates exosomal secretion [GO:1990182] References: PMID:24105262 Sources: GOC:TermGenie, GO_REF:0000058